{
  "gene": "UniProtKB:P78357",
  "term_label": "neuron projection morphogenesis",
  "gene_name": "Contactin-associated protein 1",
  "term_id": "GO:0048812",
  "gene_symbol": "CNTNAP1"
}